{
  "term_id": "GO:0005737",
  "term_label": "cytoplasm",
  "gene": "UniProtKB:O60828",
  "gene_name": "Polyglutamine-binding protein 1",
  "gene_symbol": "PQBP1"
}